alphav-beta3 integrin-CD47 complex [GO:0070357] (cellular component) Also known as: ITGB3-ITGAV-CD47 complex Relationships: is a type of plasma membrane protein complex [GO:0098797] Definition: A protein complex that consists of an alphav-beta3 integrin complex bound to CD47 (also known as IAP). References: PMID:2277087, PMID:7691831